{
  "gene_name": "Acetyl-coenzyme A synthetase 2-like, mitochondrial",
  "term_id": "GO:0005739",
  "gene_symbol": "ACSS1",
  "gene": "UniProtKB:Q9NUB1",
  "term_label": "mitochondrion"
}